{
  "gene_symbol": "CDIPTOSP",
  "term_label": "Unknown biological process",
  "term_id": "UNKNOWN:0002",
  "gene": "UniProtKB:P0DO92",
  "gene_name": "Putative protein T-ENOL"
}